{
  "gene_name": "Citrate synthase, mitochondrial",
  "term_label": "citrate synthase activity",
  "gene_symbol": "CS",
  "gene": "UniProtKB:O75390",
  "term_id": "GO:0036440"
}